{
  "term_id": "UNKNOWN:0002",
  "gene": "UniProtKB:Q0VG73",
  "gene_name": "Putative uncharacterized protein LOC152225",
  "gene_symbol": "Q0VG73",
  "term_label": "Unknown biological process"
}